leptomycin B binding [GO:1901707] (molecular function) Relationships: is a type of fatty acid binding [GO:0005504]; is a type of heterocyclic compound binding [GO:1901363] Sources: GOC:TermGenie Definition: Binding to leptomycin B.